arylsulfatase activity [GO:0004065] (molecular function) Definition: Catalysis of the reaction: a phenol sulfate + H2O = a phenol + sulfate. Sources: EC:3.1.6.1 Also known as: arylsulphatase activity, 4-methylumbelliferyl sulfatase activity, aryl-sulfate sulfohydrolase activity, aryl-sulfate sulphohydrolase activity, aryl-sulphate sulphohydrolase activity, arylsulfohydrolase activity, estrogen sulfatase activity, nitrocatechol sulfatase activity, p-nitrophenyl sulfatase activity, phenolsulfatase activity, phenylsulfatase activity, sulfatase activity Relationships: is a type of GO:0008484